{
  "gene_name": "Ubiquitin-associated protein 1-like",
  "term_id": "GO:0043130",
  "gene": "UniProtKB:F5GYI3",
  "gene_symbol": "UBAP1L",
  "term_label": "ubiquitin binding"
}